{
  "term_label": "mRNA binding",
  "term_id": "GO:0003729",
  "gene_name": "Serine_arginine-rich splicing factor 8",
  "gene": "UniProtKB:Q9BRL6",
  "gene_symbol": "SRSF8"
}